{
  "term_id": "UNKNOWN:0002",
  "gene_name": "Golgin subfamily A member 6-like protein 4",
  "gene_symbol": "GOLGA6L4",
  "term_label": "Unknown biological process",
  "gene": "UniProtKB:A6NEF3"
}